{
  "term_id": "UNKNOWN:0002",
  "gene_symbol": "MRPL14",
  "gene_name": "Large ribosomal subunit protein uL14m",
  "term_label": "Unknown biological process",
  "gene": "UniProtKB:Q6P1L8"
}